negative regulation of dauer larval development [GO:0061067] (biological process) Definition: Any process that decreases the rate, frequency, or extent of dauer larval development, the process whose specific outcome is the progression of the dauer larva over time, through the facultative diapause of the dauer (enduring) larval stage, with specialized traits adapted for dispersal and long-term survival, with elevated stress resistance and without feeding. Relationships: is a type of negative regulation of nematode larval development [GO:0061064]; is a type of regulation of dauer larval development [GO:0061065]; negatively regulates GO:0040024 Sources: GOC:dph, GOC:kmv Subtypes: negative regulation of dauer entry [GO:1905910]